{
  "term_id": "GO:0005634",
  "gene_name": "cGMP-dependent 3',5'-cyclic phosphodiesterase",
  "gene_symbol": "PDE2A",
  "gene": "UniProtKB:O00408",
  "term_label": "nucleus"
}